MHC class I protein complex assembly [GO:0002397] (biological process) References: PMID:15771591 Sources: GOC:add, ISBN:0781735149 Relationships: is a type of MHC protein complex assembly [GO:0002396] Definition: The aggregation, arrangement and bonding together of a set of components to form an MHC class I protein complex. Class I here refers to classical class I molecules.